{
  "gene_symbol": "KIF16B",
  "gene_name": "Kinesin-like protein KIF16B",
  "gene": "UniProtKB:Q96L93",
  "term_id": "GO:0047496",
  "term_label": "vesicle transport along microtubule"
}